{
  "gene_symbol": "LMOD2",
  "term_id": "GO:0006936",
  "term_label": "muscle contraction",
  "gene": "UniProtKB:Q6P5Q4",
  "gene_name": "Leiomodin-2"
}